{
  "gene": "UniProtKB:P37235",
  "gene_name": "Hippocalcin-like protein 1",
  "gene_symbol": "HPCAL1",
  "term_id": "UNKNOWN:0003",
  "term_label": "Unknown cellular component"
}